{
  "term_label": "Unknown molecular function",
  "gene_name": "Ribosomal biogenesis protein LAS1L",
  "gene_symbol": "LAS1L",
  "term_id": "UNKNOWN:0001",
  "gene": "UniProtKB:Q9Y4W2"
}